{
  "gene_symbol": "DCAF7",
  "gene_name": "DDB1- and CUL4-associated factor 7",
  "gene": "UniProtKB:P61962",
  "term_label": "Unknown biological process",
  "term_id": "UNKNOWN:0002"
}